exon-exon junction complex disassembly [GO:1903259] (biological process) References: PMID:24967911 Sources: GOC:TermGenie, GOC:sart, GO_REF:0000079 Also known as: EJC disassembly Relationships: is a type of protein-containing complex disassembly [GO:0032984] Definition: The disaggregation of an exon-exon junction complex into its constituent components.